aminoglycoside nucleotidyltransferase activity [GO:0034068] (molecular function) Definition: Catalysis of the reaction: nucleoside triphosphate + aminoglycoside = diphosphate + nucleotidylaminoglycoside. Also known as: aminoglycoside adenylyltransferase activity, streptomycin adenylate synthetase activity, streptomycin adenyltransferase activity, streptomycin adenylylase activity, streptomycin adenylyltransferase activity, streptomycin-spectinomycin adenylyltransferase activity Relationships: is a type of nucleotidyltransferase activity [GO:0016779] Subtypes: GO:0008871, aminoglycoside 3''-adenylyltransferase activity [GO:0009012] Sources: GOC:cb